{
  "gene": "UniProtKB:A4FU69",
  "gene_name": "EF-hand calcium-binding domain-containing protein 5",
  "term_id": "UNKNOWN:0001",
  "gene_symbol": "EFCAB5",
  "term_label": "Unknown molecular function"
}